positive regulation of intracellular signal transduction [GO:1902533] (biological process) Definition: Any process that activates or increases the frequency, rate or extent of intracellular signal transduction. Sources: GOC:BHF, GOC:TermGenie, GOC:dph, GOC:signaling, GOC:tb Also known as: positive regulation of intracellular signaling chain, up regulation of intracellular signal transduction, up regulation of intracellular signaling chain, up-regulation of intracellular signal transduction, up-regulation of intracellular signaling chain, upregulation of intracellular signal transduction, upregulation of intracellular signaling chain, activation of intracellular signal transduction, activation of intracellular signal transduction pathway, activation of intracellular signaling cascade, activation of intracellular signaling chain, activation of signal transmission via intracellular cascade, positive regulation of intracellular protein kinase cascade, positive regulation of intracellular signal transduction pathway, positive regulation of signal transmission via intracellular cascade, up regulation of intracellular signal transduction pathway, up regulation of signal transmission via intracellular cascade, up-regulation of intracellular signal transduction pathway, up-regulation of signal transmission via intracellular cascade, upregulation of intracellular signal transduction pathway, upregulation of signal transmission via intracellular cascade, activation of intracellular signaling pathway, activation of signal transduction via intracellular signaling cascade, positive regulation of intracellular signaling cascade, positive regulation of intracellular signaling pathway, positive regulation of signal transduction via intracellular signaling cascade, up regulation of intracellular signaling cascade, up regulation of intracellular signaling pathway, up regulation of signal transduction via intracellular signaling cascade, up-regulation of intracellular signaling cascade, up-regulation of intracellular signaling pathway, up-regulation of signal transduction via intracellular signaling cascade, upregulation of intracellular signaling cascade, upregulation of intracellular signaling pathway, upregulation of signal transduction via intracellular signaling cascade Relationships: is a type of GO:0009967; is_a regulation of intracellular signal transduction [GO:1902531]; positively regulates intracellular signal transduction [GO:0035556] Subtypes: positive regulation of thyroid hormone receptor signaling pathway [GO:0002157], GO:0010750, GO:0032008, positive regulation of intracellular steroid hormone receptor signaling pathway [GO:0033145], GO:0034141, positive regulation of toll-like receptor 7 signaling pathway [GO:0034157], positive regulation of toll-like receptor 8 signaling pathway [GO:0034161], positive regulation of toll-like receptor 9 signaling pathway [GO:0034165], positive regulation of toll-like receptor 11 signaling pathway [GO:0034173], positive regulation of toll-like receptor 12 signaling pathway [GO:0034177], GO:0034181, positive regulation of hippo signaling [GO:0035332], GO:0035360, positive regulation of canonical NF-kappaB signal transduction [GO:0043123], positive regulation of MAPK cascade [GO:0043410], positive regulation of retinoic acid receptor signaling pathway [GO:0048386], positive regulation of calcium-mediated signaling [GO:0050850], positive regulation of small GTPase mediated signal transduction [GO:0051057], positive regulation of phosphatidylinositol 3-kinase/protein kinase B signal transduction [GO:0051897], GO:0060391, positive regulation of phosphorelay signal transduction system [GO:0070299], GO:0070304, positive regulation of nucleotide-binding domain, leucine rich repeat containing receptor signaling pathway [GO:0070426], positive regulation of vitamin D receptor signaling pathway [GO:0070564], GO:0090037, GO:0141087, GO:0141111, GO:0141163, GO:0141214, positive regulation of endoplasmic reticulum unfolded protein response [GO:1900103], positive regulation of MDA-5 signaling pathway [GO:1900245], positive regulation of RIG-I signaling pathway [GO:1900246], positive regulation of non-canonical NF-kappaB signal transduction [GO:1901224], positive regulation of signal transduction by p53 class mediator [GO:1901798], GO:1901978, GO:1902073, positive regulation of SREBP signaling pathway [GO:2000640], positive regulation of intrinsic apoptotic signaling pathway [GO:2001244]